cellular response to butyrate [GO:1903545] (biological process) Definition: Any process that results in a change in state or activity of a cell (in terms of movement, secretion, enzyme production, gene expression, etc.) as a result of a butyrate stimulus. Relationships: is a type of cellular response to fatty acid [GO:0071398]; is a type of response to butyrate [GO:1903544] References: PMID:9734870 Sources: GOC:TermGenie, GOC:mr, GO_REF:0000071